CRD domain binding [GO:0071906] (molecular function) Relationships: is a type of protein domain specific binding [GO:0019904] Also known as: context dependent regulatory domain binding Definition: Binding to a CRD (context dependent regulatory) domain, a domain of about 130 residues that is the most divergent region among the LEF/TCF proteins. References: PMID:19460168 Sources: GOC:yaf